spore dispersal [GO:0075325] (biological process) Relationships: is a type of reproductive process [GO:0022414] Also known as: spore dispersal on or near host during symbiotic interaction, active spore dispersal on or near host, active spore dispersal on or near host during symbiotic interaction, passive spore dispersal on or near host, spore dispersal on or near host Definition: Any process in which an organism disseminates its spores. Sources: Wikipedia:Spore